aromatase activity [GO:0070330] (molecular function) Sources: EC:1.14.14.14 Relationships: is a type of GO:0016712 Definition: Catalysis of the reaction: 3 O2 + 3 reduced [NADPH--hemoprotein reductase] + testosterone = 17beta-estradiol + formate + 4 H+ + 4 H2O + 3 oxidized [NADPH--hemoprotein reductase]. Also converts androst-4-ene-3,17-dione into estrone. Also known as: estrogen synthetase activity